{
  "gene": "UniProtKB:P0CG48",
  "gene_name": "Polyubiquitin-C",
  "gene_symbol": "UBC",
  "term_label": "protein ubiquitination",
  "term_id": "GO:0016567"
}